branched-chain alpha-keto acid decarboxylation to branched-chain acyl-CoA [GO:0120552] (biological process) Definition: The chemical reactions and pathways resulting in the formation of a branched-chain acyl-CoA by the oxidative decarboxylation of a branched-chain alpha-keto acid derived from L-leucine, L-isoleucine or L-valine. This pathway comprises a series of three reactions carried out by a multisubunit complex called the 'branched-chain alpha-keto acid dehydrogenase complex', even though branched-chain alpha-keto acid dehydrogenase activity describes only one of those reactions. The combination of the three reactions can be summarized as: 3-methyl-2-oxobutanoate + coenzyme A + NAD+ -> branched-chain acyl-CoA + CO2 + NADH. Specific substrates include 3-methyl-2-oxobutanoate (a transamination product of L-valine), (S)-3-methyl-2-oxopentanoate (a transamination product of L-isoleucine) and 4-methyl-2-oxopentanoate (a transamination product of L-leucine), which generate the products 2-methylpropanoyl-CoA, 2-methylbutanoyl-CoA and 3-methylbutanoyl-CoA, respectively. Sources: MetaCyc:PWY-5046 Also known as: branched-chain 2-oxo acid dehydrogenase system, branched-chain alpha-keto acid dehydrogenase system Relationships: is a type of carboxylic acid metabolic process [GO:0019752]; is a type of GO:0035337; is part of branched-chain amino acid catabolic process [GO:0009083]